{
  "gene_symbol": "HSD11B1",
  "term_id": "GO:0070524",
  "term_label": "11-beta-hydroxysteroid dehydrogenase (NADP+) activity",
  "gene_name": "11-beta-hydroxysteroid dehydrogenase 1",
  "gene": "UniProtKB:P28845"
}